{
  "gene_symbol": "MYF5",
  "term_label": "Unknown cellular component",
  "gene_name": "Myogenic factor 5",
  "term_id": "UNKNOWN:0003",
  "gene": "UniProtKB:P13349"
}